{
  "gene_name": "Rac GTPase-activating protein 1",
  "term_label": "midbody",
  "term_id": "GO:0030496",
  "gene": "UniProtKB:Q9H0H5",
  "gene_symbol": "RACGAP1"
}